{
  "gene_symbol": "TEDC2",
  "term_label": "Unknown molecular function",
  "gene": "UniProtKB:Q7L2K0",
  "gene_name": "Tubulin epsilon and delta complex protein 2",
  "term_id": "UNKNOWN:0001"
}